cellular response to papulacandin B [GO:0072731] (BP) Relationships: is a type of GO:0071396; is_a response to papulacandin B [GO:0072730]; is a type of cellular response to oxygen-containing compound [GO:1901701] Sources: GOC:mah Definition: Any process that results in a change in state or activity of a cell (in terms of movement, secretion, enzyme production, gene expression, etc.) as a result of a papulacandin B stimulus.